{
  "term_id": "GO:0005615",
  "gene_name": "C-C motif chemokine 27",
  "term_label": "extracellular space",
  "gene": "UniProtKB:Q9Y4X3",
  "gene_symbol": "CCL27"
}